{
  "gene_symbol": "KANK3",
  "term_label": "negative regulation of actin filament polymerization",
  "gene": "UniProtKB:Q6NY19",
  "term_id": "GO:0030837",
  "gene_name": "KN motif and ankyrin repeat domain-containing protein 3"
}